{
  "term_id": "GO:0035249",
  "gene": "UniProtKB:Q12879",
  "term_label": "synaptic transmission, glutamatergic",
  "gene_name": "Glutamate receptor ionotropic, NMDA 2A",
  "gene_symbol": "GRIN2A"
}